{
  "gene": "UniProtKB:Q5VVH2",
  "gene_symbol": "FKBP1C",
  "term_id": "GO:0010881",
  "gene_name": "Peptidyl-prolyl cis-trans isomerase FKBP1C",
  "term_label": "regulation of cardiac muscle contraction by regulation of the release of sequestered calcium ion"
}